{
  "gene_name": "Poly-ADP-ribosylation-amplifying and CtIP-maintaining micropeptide",
  "term_id": "UNKNOWN:0002",
  "gene_symbol": "MARCHF6-DT",
  "term_label": "Unknown biological process",
  "gene": "UniProtKB:P0DW81"
}